{
  "term_label": "inflammatory response",
  "gene_symbol": "FPR1",
  "gene_name": "fMet-Leu-Phe receptor",
  "gene": "UniProtKB:P21462",
  "term_id": "GO:0006954"
}